{
  "gene_symbol": "WNT9A",
  "term_label": "extracellular space",
  "term_id": "GO:0005615",
  "gene": "UniProtKB:O14904",
  "gene_name": "Protein Wnt-9a"
}